synapsis initiation complex [GO:0106069] (cellular component) References: PMID:16847351 Definition: A SUMO-E3 ligase complex capable of promoting synapsis, the meiotic cell cycle process where side by side pairing and physical juxtaposition of homologous chromosomes is created during meiotic prophase. Relationships: is a type of SUMO ligase complex [GO:0106068]; is a type of nuclear protein-containing complex [GO:0140513]; is part of condensed nuclear chromosome [GO:0000794]